{
  "gene_symbol": "H2BK1",
  "term_label": "structural constituent of chromatin",
  "gene": "UniProtKB:A0A2R8Y619",
  "term_id": "GO:0030527",
  "gene_name": "Histone H2B type 2-K1"
}